{
  "gene_symbol": "VAX1",
  "gene_name": "Ventral anterior homeobox 1",
  "gene": "UniProtKB:Q5SQQ9",
  "term_label": "neuron differentiation",
  "term_id": "GO:0030182"
}